regulation of homophilic cell adhesion [GO:1903385] (BP) Definition: Any process that modulates the frequency, rate or extent of homophilic cell adhesion. References: PMID:21724833 Sources: GOC:TermGenie, GOC:als, GO_REF:0000058 Relationships: is a type of regulation of cell-cell adhesion [GO:0022407]; regulates homophilic cell-cell adhesion [GO:0007156] Subtypes: negative regulation of homophilic cell adhesion [GO:1903386], GO:1903387